{
  "term_id": "GO:0005886",
  "term_label": "plasma membrane",
  "gene_symbol": "PALLD",
  "gene": "UniProtKB:Q8WX93",
  "gene_name": "Palladin"
}